central vacuole [GO:0042807] (cellular component) Sources: ISBN:9780815341116, Wikipedia:Vacuole Relationships: is a type of GO:0000325 Definition: A membrane-enclosed sac that takes up most of the volume of a mature plant cell. Functions include storage, separation of toxic byproducts, and cell growth determination.